{
  "gene_name": "Serine_threonine-protein phosphatase 2A 65 kDa regulatory subunit A beta isoform",
  "gene_symbol": "PPP2R1B",
  "term_id": "GO:0005634",
  "gene": "UniProtKB:P30154",
  "term_label": "nucleus"
}